double-stranded/single-stranded junction telomeric DNA binding [GO:0090655] (molecular function) Relationships: is a type of double-strand/single-strand DNA junction binding [GO:0000406]; is_a telomeric DNA binding [GO:0042162] References: PMID:21852327 Sources: GOC:BHF, GOC:BHF_telomere, GOC:bhm, GOC:nc Definition: Binding to a junction formed at the point where double-stranded telomeric DNA becomes a single-stranded G-rich telomeric DNA 3' overhang.